{
  "term_id": "UNKNOWN:0002",
  "gene_name": "Uncharacterized protein encoded by LINC01548",
  "gene": "UniProtKB:A6NM66",
  "term_label": "Unknown biological process",
  "gene_symbol": "LINC01548"
}